{
  "term_id": "GO:0071014",
  "term_label": "post-mRNA release spliceosomal complex",
  "gene_symbol": "XAB2",
  "gene_name": "Pre-mRNA-splicing factor SYF1",
  "gene": "UniProtKB:Q9HCS7"
}